{
  "term_id": "GO:0006955",
  "gene_name": "Immunoglobulin kappa variable 2-30",
  "term_label": "immune response",
  "gene": "UniProtKB:P06310",
  "gene_symbol": "IGKV2-30"
}